{
  "term_label": "Unknown molecular function",
  "gene_symbol": "ZCCHC12",
  "term_id": "UNKNOWN:0001",
  "gene": "UniProtKB:Q6PEW1",
  "gene_name": "Zinc finger CCHC domain-containing protein 12"
}